positive regulation of memory T cell activation [GO:2000568] (biological process) Relationships: is a type of positive regulation of T cell activation [GO:0050870]; is a type of regulation of memory T cell activation [GO:2000567]; positively regulates memory T cell activation [GO:0035709] Sources: GOC:obol Definition: Any process that activates or increases the frequency, rate or extent of memory T cell activation.